{
  "gene_name": "DENN domain-containing protein 1B",
  "gene_symbol": "DENND1B",
  "term_label": "nuclear speck",
  "term_id": "GO:0016607",
  "gene": "UniProtKB:Q6P3S1"
}